{
  "gene_symbol": "VDR",
  "term_label": "vitamin D binding",
  "term_id": "GO:0005499",
  "gene_name": "Vitamin D3 receptor",
  "gene": "UniProtKB:P11473"
}